{
  "term_id": "GO:0005930",
  "gene_symbol": "CCDC39",
  "gene_name": "Coiled-coil domain-containing protein 39",
  "term_label": "axoneme",
  "gene": "UniProtKB:Q9UFE4"
}